IRE1-TRAF2-ASK1 complex [GO:1990604] (cellular component) Also known as: ERN1-TRAF2-ASK1 complex Definition: A protein complex of the endoplasmic reticulum membrane that consists of IRE1 (Inositol-requiring enzyme-1), TRAF2 (TNF receptor-associated factor 2) and ASK1 (Apoptosis signal-regulating kinase 1, a MAP3K). Relationships: is a type of membrane protein complex [GO:0098796]; is a type of endoplasmic reticulum protein-containing complex [GO:0140534]; is part of GO:0005789 References: PMID:12050113, PMID:23000344 Sources: GOC:PARL, GOC:bf